{
  "gene_name": "Major facilitator superfamily domain-containing protein 12",
  "term_label": "cysteine transmembrane transporter activity",
  "gene": "UniProtKB:Q6NUT3",
  "term_id": "GO:0033229",
  "gene_symbol": "MFSD12"
}